{
  "term_label": "cytoplasm",
  "term_id": "GO:0005737",
  "gene_name": "NEDD8-activating enzyme E1 catalytic subunit",
  "gene": "UniProtKB:Q8TBC4",
  "gene_symbol": "UBA3"
}